{
  "gene_symbol": "OAT",
  "gene": "UniProtKB:P04181",
  "gene_name": "Ornithine aminotransferase, mitochondrial",
  "term_label": "L-arginine catabolic process to proline via ornithine",
  "term_id": "GO:0010121"
}